{
  "term_label": "Unknown biological process",
  "term_id": "UNKNOWN:0002",
  "gene_name": "Phytanoyl-CoA hydroxylase-interacting protein",
  "gene": "UniProtKB:Q92561",
  "gene_symbol": "PHYHIP"
}